{
  "gene_name": "Helicase ARIP4",
  "term_id": "GO:0003712",
  "gene": "UniProtKB:Q9Y4B4",
  "gene_symbol": "RAD54L2",
  "term_label": "transcription coregulator activity"
}